Malpighian tubule tip cell differentiation [GO:0061382] (biological process) References: PMID:7821213 Sources: GOC:dph, GOC:mtg_kidney_jan10 Definition: The process in which a relatively unspecialized cell acquires specialized features of a Malpighian tubule tip cell. A Malpighian tubule tip cell is a mitogenic signaling cell that controls the proliferation of its neighboring cells. Relationships: is a type of GO:0030154; BFO_0000050 Malpighian tubule development [GO:0072002]